L-allo-threonine aldolase activity [GO:0008732] (molecular function) Definition: Catalysis of the reaction: L-allo-threonine = glycine + acetaldehyde. Relationships: is a type of threonine aldolase activity [GO:0004793] Also known as: L-allo-threonine acetaldehyde-lyase activity, LtaA References: PMID:9228760 Sources: RHEA:26209